{
  "gene_name": "Intercellular adhesion molecule 2",
  "gene": "UniProtKB:P13598",
  "term_id": "GO:0005886",
  "gene_symbol": "ICAM2",
  "term_label": "plasma membrane"
}